galacturan 1,4-alpha-galacturonidase activity [GO:0047911] (molecular function) Relationships: is a type of hydrolase activity, hydrolyzing O-glycosyl compounds [GO:0004553] Also known as: exo-D-galacturonase activity, exo-polygalacturonase activity, exopoly-D-galacturonase activity, galacturan alpha-1,4-galacturonidase activity, exo-D-galacturonanase activity, exopolygalacturonase activity, poly(1,4-alpha-D-galacturonide) galacturonohydrolase activity, poly(galacturonate) hydrolase activity Sources: EC:3.2.1.67, MetaCyc:GALACTURAN-14-ALPHA-GALACTURONIDASE-RXN Definition: Catalysis of the reaction: [(1->4)-alpha-D-galacturonide](n) + H2O = [(1->4)-alpha-D-galacturonide](n-1) + D-galacturonate.